{
  "term_id": "GO:0003924",
  "gene_symbol": "GIMAP2",
  "gene_name": "GTPase IMAP family member 2",
  "gene": "UniProtKB:Q9UG22",
  "term_label": "GTPase activity"
}